{
  "gene_name": "Vesicle transport protein SFT2A",
  "term_label": "Unknown molecular function",
  "term_id": "UNKNOWN:0001",
  "gene_symbol": "SFT2D1",
  "gene": "UniProtKB:Q8WV19"
}